{
  "term_label": "terminal bouton",
  "term_id": "GO:0043195",
  "gene_name": "Neuromedin-U",
  "gene_symbol": "NMU",
  "gene": "UniProtKB:P48645"
}